{
  "term_label": "Unknown cellular component",
  "gene_name": "Neurexophilin-2",
  "term_id": "UNKNOWN:0003",
  "gene": "UniProtKB:O95156",
  "gene_symbol": "NXPH2"
}